{
  "gene_symbol": "PPIAL4G",
  "term_label": "cyclosporin A binding",
  "gene": "UniProtKB:P0DN37",
  "gene_name": "Peptidyl-prolyl cis-trans isomerase A-like 4G",
  "term_id": "GO:0016018"
}